{
  "gene_name": "Cyclin-dependent kinases regulatory subunit 1",
  "term_id": "GO:0019005",
  "term_label": "SCF ubiquitin ligase complex",
  "gene_symbol": "CKS1B",
  "gene": "UniProtKB:P61024"
}